{
  "gene_symbol": "PMCHL2",
  "gene_name": "Putative pro-MCH-like protein 2",
  "term_label": "type 1 melanin-concentrating hormone receptor binding",
  "term_id": "GO:0031777",
  "gene": "UniProtKB:Q9BQD1"
}